{
  "term_label": "centrosome",
  "gene": "UniProtKB:P0DP23",
  "gene_symbol": "CALM1",
  "term_id": "GO:0005813",
  "gene_name": "Calmodulin-1"
}